{
  "gene_name": "Spindle and kinetochore-associated protein 3",
  "gene": "UniProtKB:Q8IX90",
  "term_label": "mitotic cell cycle",
  "term_id": "GO:0000278",
  "gene_symbol": "SKA3"
}